{
  "gene_name": "HLA class I histocompatibility antigen, C alpha chain",
  "term_label": "peptide antigen binding",
  "term_id": "GO:0042605",
  "gene": "UniProtKB:P10321",
  "gene_symbol": "HLA-C"
}